monoatomic anion homeostasis [GO:0055081] (biological process) Subtypes: GO:0030002, chloride ion homeostasis [GO:0055064] Sources: GOC:ceb, GOC:jid, GOC:mah Relationships: is a type of monoatomic ion homeostasis [GO:0050801] Definition: Any process involved in the maintenance of an internal steady state of monoatomic anions within an organism or cell. Monatomic anions (also called simple anions) are anions consisting of exactly one atom. Also known as: anion homeostasis